{
  "term_label": "nucleus",
  "gene_name": "Zinc finger protein 577",
  "gene_symbol": "ZNF577",
  "term_id": "GO:0005634",
  "gene": "UniProtKB:Q9BSK1"
}